{
  "gene_name": "T cell receptor alpha joining 30 (Fragment)",
  "gene_symbol": "TRAJ30",
  "term_label": "Unknown biological process",
  "gene": "UniProtKB:A0A075B6Y1",
  "term_id": "UNKNOWN:0002"
}